{
  "gene_name": "Adenomatous polyposis coli protein",
  "gene_symbol": "APC",
  "term_id": "GO:0030877",
  "gene": "UniProtKB:P25054",
  "term_label": "beta-catenin destruction complex"
}